{
  "term_id": "GO:0005576",
  "gene_symbol": "SPRR2A",
  "gene_name": "Small proline-rich protein 2A",
  "term_label": "extracellular region",
  "gene": "UniProtKB:P35326"
}